{
  "gene": "UniProtKB:Q9BYR7",
  "term_label": "Unknown cellular component",
  "term_id": "UNKNOWN:0003",
  "gene_symbol": "KRTAP3-2",
  "gene_name": "Keratin-associated protein 3-2"
}